{
  "term_id": "GO:0006783",
  "gene": "UniProtKB:P08397",
  "term_label": "heme biosynthetic process",
  "gene_symbol": "HMBS",
  "gene_name": "Porphobilinogen deaminase"
}